{
  "gene_symbol": "ASXL1",
  "term_id": "GO:0045944",
  "gene_name": "Polycomb group protein ASXL1",
  "gene": "UniProtKB:Q8IXJ9",
  "term_label": "positive regulation of transcription by RNA polymerase II"
}